{
  "gene_symbol": "KCNA2",
  "term_label": "potassium ion transmembrane transport",
  "term_id": "GO:0071805",
  "gene": "UniProtKB:P16389",
  "gene_name": "Potassium voltage-gated channel subfamily A member 2"
}